{
  "term_label": "Unknown cellular component",
  "gene_name": "Protein canopy homolog 3",
  "gene": "UniProtKB:Q9BT09",
  "term_id": "UNKNOWN:0003",
  "gene_symbol": "CNPY3"
}